{
  "gene_name": "NUT family member 2B",
  "gene_symbol": "NUTM2B",
  "term_label": "Unknown biological process",
  "gene": "UniProtKB:A6NNL0",
  "term_id": "UNKNOWN:0002"
}